{
  "term_id": "GO:0004382",
  "gene_symbol": "ENTPD8",
  "term_label": "GDP phosphatase activity",
  "gene": "UniProtKB:Q5MY95",
  "gene_name": "Ectonucleoside triphosphate diphosphohydrolase 8"
}